{
  "term_id": "GO:0005085",
  "gene": "UniProtKB:Q9NRD0",
  "gene_name": "F-box only protein 8",
  "term_label": "guanyl-nucleotide exchange factor activity",
  "gene_symbol": "FBXO8"
}